{
  "term_id": "GO:0045104",
  "gene": "UniProtKB:Q9UPN3",
  "term_label": "intermediate filament cytoskeleton organization",
  "gene_name": "Microtubule-actin cross-linking factor 1, isoforms 1_2_3_4_5",
  "gene_symbol": "MACF1"
}